{
  "gene": "UniProtKB:P48059",
  "term_id": "GO:0005737",
  "gene_symbol": "LIMS1",
  "term_label": "cytoplasm",
  "gene_name": "LIM and senescent cell antigen-like-containing domain protein 1"
}